{
  "term_id": "GO:0004878",
  "gene_name": "C3a anaphylatoxin chemotactic receptor",
  "gene_symbol": "C3AR1",
  "gene": "UniProtKB:Q16581",
  "term_label": "complement component C5a receptor activity"
}